{
  "gene_name": "Immunoglobulin heavy diversity 3-9 (Fragment)",
  "gene_symbol": "IGHD3-9",
  "term_label": "Unknown cellular component",
  "term_id": "UNKNOWN:0003",
  "gene": "UniProtKB:A0A0J9YW22"
}